{
  "term_id": "UNKNOWN:0002",
  "gene_symbol": "NXPH1",
  "term_label": "Unknown biological process",
  "gene_name": "Neurexophilin-1",
  "gene": "UniProtKB:P58417"
}